{
  "term_label": "Unknown molecular function",
  "gene_symbol": "CYS1",
  "term_id": "UNKNOWN:0001",
  "gene": "UniProtKB:Q717R9",
  "gene_name": "Cystin-1"
}